{
  "gene_name": "POTE ankyrin domain family member F",
  "gene": "UniProtKB:A5A3E0",
  "gene_symbol": "POTEF",
  "term_id": "GO:0015629",
  "term_label": "actin cytoskeleton"
}